{
  "gene": "UniProtKB:P19447",
  "term_id": "GO:0005675",
  "gene_symbol": "ERCC3",
  "term_label": "transcription factor TFIIH holo complex",
  "gene_name": "General transcription and DNA repair factor IIH helicase subunit XPB"
}